chemotaxis to folate [GO:0043326] (biological process) Definition: The directed movement of a motile cell or organism in response to the presence of folate. Relationships: is a type of chemotaxis [GO:0006935]; is a type of response to folic acid [GO:0051593] Sources: GOC:go_curators